{
  "term_id": "UNKNOWN:0002",
  "gene": "UniProtKB:Q7Z4W2",
  "gene_symbol": "LYZL2",
  "term_label": "Unknown biological process",
  "gene_name": "Lysozyme-like protein 2"
}